lytic vacuole [GO:0000323] (cellular component) Relationships: is a type of GO:0005773 Sources: GOC:krc Definition: A vacuole that is maintained at an acidic pH and which contains degradative enzymes, including a wide variety of acid hydrolases. Subtypes: GO:0000324, lytic vacuole within protein storage vacuole [GO:0000327], GO:0005764, senescence-associated vacuole [GO:0010282], reservosome [GO:0106123]